stereocilium bundle [GO:0032421] (cellular component) References: PMID:15661519, PMID:7840137 Sources: GOC:ecd Relationships: is_a GO:0098862; has part GO:0032420 Also known as: stereocilia bundle Definition: A bundle of cross-linked stereocilia, arranged around a kinocilium on the apical surface of a sensory hair cell (e.g. a neuromast, auditory or vestibular hair cell). Stereocilium bundles act as mechanosensory organelles by responding to fluid motion or fluid pressure changes.